{
  "gene_symbol": "KANK4",
  "term_label": "negative regulation of actin filament polymerization",
  "gene_name": "KN motif and ankyrin repeat domain-containing protein 4",
  "term_id": "GO:0030837",
  "gene": "UniProtKB:Q5T7N3"
}